negative regulation of hair cycle [GO:0042636] (biological process) Definition: Any process that stops, prevents, or reduces the frequency, rate or extent of the cyclical phases of growth (anagen), regression (catagen), quiescence (telogen), and shedding (exogen) in the life of a hair. References: PMID:12230507 Sources: GOC:go_curators Also known as: down regulation of hair cycle, down-regulation of hair cycle, downregulation of hair cycle, inhibition of hair cycle Relationships: is a type of GO:0042634; is a type of GO:0051241; negatively regulates GO:0042633